{
  "gene_symbol": "NDUFA4",
  "term_id": "GO:0045277",
  "term_label": "respiratory chain complex IV",
  "gene_name": "Cytochrome c oxidase subunit NDUFA4",
  "gene": "UniProtKB:O00483"
}